{
  "term_label": "lipid binding",
  "term_id": "GO:0008289",
  "gene_name": "Testis-expressed protein 2",
  "gene_symbol": "TEX2",
  "gene": "UniProtKB:Q8IWB9"
}